{
  "term_label": "virus receptor activity",
  "gene_name": "C-type lectin domain family 5 member A",
  "term_id": "GO:0001618",
  "gene_symbol": "CLEC5A",
  "gene": "UniProtKB:Q9NY25"
}